{
  "gene_symbol": "CLCF1",
  "term_id": "UNKNOWN:0001",
  "term_label": "Unknown molecular function",
  "gene_name": "Cardiotrophin-like cytokine factor 1",
  "gene": "UniProtKB:Q9UBD9"
}